{
  "term_label": "mitochondrion transport along microtubule",
  "gene_symbol": "RHOT2",
  "gene": "UniProtKB:Q8IXI1",
  "term_id": "GO:0047497",
  "gene_name": "Mitochondrial Rho GTPase 2"
}